{
  "gene": "UniProtKB:Q9Y2P4",
  "gene_name": "Long-chain fatty acid transport protein 6",
  "gene_symbol": "SLC27A6",
  "term_id": "GO:0001676",
  "term_label": "long-chain fatty acid metabolic process"
}